{
  "gene_name": "Translation initiation factor IF-2, mitochondrial",
  "term_label": "mitochondrial translational initiation",
  "term_id": "GO:0070124",
  "gene": "UniProtKB:P46199",
  "gene_symbol": "MTIF2"
}